protein localization to growing cell tip [GO:1902486] (biological process) Definition: A process in which a protein is transported to, or maintained in, a location within a growing cell tip. Also known as: protein localisation in growing cell tip, protein localisation to growing cell tip, protein localization in growing cell tip References: PMID:23041194 Sources: GOC:TermGenie Relationships: is a type of GO:1990151 Subtypes: protein localization to old growing cell tip [GO:1903858], protein localization to new growing cell tip [GO:1904758]